{
  "gene": "UniProtKB:Q6ZMC9",
  "gene_name": "Sialic acid-binding Ig-like lectin 15",
  "term_label": "plasma membrane",
  "term_id": "GO:0005886",
  "gene_symbol": "SIGLEC15"
}